stemar-13-ene synthase activity [GO:0034278] (molecular function) Relationships: is a type of carbon-oxygen lyase activity, acting on phosphates [GO:0016838] Also known as: 9alpha-copalyl-diphosphate diphosphate-lyase (stemar-13-ene-forming) activity Definition: Catalysis of the reaction: 9-alpha-copalyl diphosphate = stemar-13-ene + diphosphate. Sources: RHEA:25552